{
  "gene_name": "Homeobox protein Hox-C13",
  "term_id": "GO:0000978",
  "gene": "UniProtKB:P31276",
  "gene_symbol": "HOXC13",
  "term_label": "RNA polymerase II cis-regulatory region sequence-specific DNA binding"
}